{
  "gene_name": "Syntaxin-4",
  "gene": "UniProtKB:Q12846",
  "gene_symbol": "STX4",
  "term_id": "GO:0006906",
  "term_label": "vesicle fusion"
}